{
  "term_label": "receptor ligand activity",
  "gene_name": "Gremlin-2",
  "gene_symbol": "GREM2",
  "term_id": "GO:0048018",
  "gene": "UniProtKB:Q9H772"
}